{
  "term_label": "Unknown biological process",
  "term_id": "UNKNOWN:0002",
  "gene_name": "Olfactory receptor 51G2",
  "gene": "UniProtKB:Q8NGK0",
  "gene_symbol": "OR51G2"
}